{
  "term_label": "calcium ion binding",
  "gene_symbol": "CALR",
  "gene": "UniProtKB:P27797",
  "gene_name": "Calreticulin",
  "term_id": "GO:0005509"
}